{
  "term_label": "regulation of Arp2/3 complex-mediated actin nucleation",
  "gene_name": "F-actin-uncapping protein LRRC16A",
  "gene": "UniProtKB:Q5VZK9",
  "gene_symbol": "CARMIL1",
  "term_id": "GO:0034315"
}